negative regulation of bioluminescence [GO:1905086] (biological process) Definition: Any process that stops, prevents or reduces the frequency, rate or extent of bioluminescence. References: PMID:10913092 Sources: GOC:BHF, GOC:TermGenie, GOC:rph, GO_REF:0000058 Also known as: down regulation of bioluminescence, down-regulation of bioluminescence, downregulation of bioluminescence, inhibition of bioluminescence Relationships: is_a negative regulation of metabolic process [GO:0009892]; is a type of regulation of bioluminescence [GO:1905085]; negatively regulates bioluminescence [GO:0008218]